{
  "gene": "UniProtKB:Q9H116",
  "term_id": "UNKNOWN:0003",
  "gene_name": "GDNF-inducible zinc finger protein 1",
  "gene_symbol": "GZF1",
  "term_label": "Unknown cellular component"
}